{
  "gene": "UniProtKB:Q96RD6",
  "gene_symbol": "PANX2",
  "gene_name": "Pannexin-2",
  "term_label": "cell-cell signaling",
  "term_id": "GO:0007267"
}